{
  "gene_name": "[Pyruvate dehydrogenase (acetyl-transferring)] kinase isozyme 2, mitochondrial",
  "term_label": "regulation of glucose metabolic process",
  "term_id": "GO:0010906",
  "gene_symbol": "PDK2",
  "gene": "UniProtKB:Q15119"
}